{
  "gene_symbol": "ACP4",
  "term_label": "regulation of neuronal synaptic plasticity",
  "term_id": "GO:0048168",
  "gene_name": "Testicular acid phosphatase",
  "gene": "UniProtKB:Q9BZG2"
}